{
  "gene_symbol": "OR5D18",
  "gene": "UniProtKB:Q8NGL1",
  "term_id": "GO:0007608",
  "gene_name": "Olfactory receptor 5D18",
  "term_label": "sensory perception of smell"
}